{
  "gene": "UniProtKB:P17542",
  "gene_symbol": "TAL1",
  "term_label": "RNA polymerase II cis-regulatory region sequence-specific DNA binding",
  "term_id": "GO:0000978",
  "gene_name": "T-cell acute lymphocytic leukemia protein 1"
}